{
  "gene_symbol": "TSLP",
  "term_id": "GO:0032733",
  "gene": "UniProtKB:Q969D9",
  "gene_name": "Thymic stromal lymphopoietin",
  "term_label": "positive regulation of interleukin-10 production"
}